{
  "term_label": "activin receptor binding",
  "term_id": "GO:0070697",
  "gene_name": "Cryptic family protein 1B",
  "gene_symbol": "CFC1B",
  "gene": "UniProtKB:P0CG36"
}